negative regulation of transmembrane transport [GO:0034763] (biological process) Definition: Any process that stops, prevents, or reduces the frequency, rate or extent of the directed movement of a solute from one side of a membrane to the other. Sources: GOC:mah Also known as: down regulation of transmembrane transport, down-regulation of transmembrane transport, downregulation of transmembrane transport, negative regulation of membrane transport, inhibition of transmembrane transport Relationships: is a type of regulation of transmembrane transport [GO:0034762]; is a type of GO:0048523; is a type of negative regulation of transport [GO:0051051]; negatively regulates GO:0055085 Subtypes: GO:0002037, negative regulation of long-chain fatty acid import across plasma membrane [GO:0010748], negative regulation of D-glucose transmembrane transport [GO:0010829], GO:0034766, negative regulation of gluconate transmembrane transport [GO:0035431], negative regulation of glycerol transport [GO:0090373], negative regulation of post-translational protein targeting to membrane, translocation [GO:0120236], negative regulation of D-aspartate import across plasma membrane [GO:0140216], negative regulation of glycine import across plasma membrane [GO:1900924], GO:1900927, negative regulation of L-tyrosine import across plasma membrane [GO:1900930], negative regulation of L-glutamine import across plasma membrane [GO:1901035], negative regulation of polyamine transmembrane transport [GO:1902268], GO:1902273, GO:1902835, negative regulation of L-lysine import across plasma membrane [GO:1905009], negative regulation of uracil import across plasma membrane [GO:1905530], negative regulation of L-leucine import across plasma membrane [GO:1905533], negative regulation of L-arginine import across plasma membrane [GO:1905542], negative regulation of L-methionine import across plasma membrane [GO:1905625], GO:1905700, negative regulation of phosphate transmembrane transport [GO:2000186], GO:2001149